hypotaurocyamine kinase activity [GO:0047715] (molecular function) Sources: EC:2.7.3.6, RHEA:24008 Also known as: ATP:hypotaurocyamine N-phosphotransferase activity Relationships: is a type of kinase activity [GO:0016301]; is a type of phosphotransferase activity, nitrogenous group as acceptor [GO:0016775] Definition: Catalysis of the reaction: ATP + hypotaurocyamine = N(omega)-phosphohypotaurocyamine + ADP + 2 H+.